{
  "gene_name": "Interleukin-5 receptor subunit alpha",
  "term_label": "receptor complex",
  "gene_symbol": "IL5RA",
  "gene": "UniProtKB:Q01344",
  "term_id": "GO:0043235"
}